{
  "gene_symbol": "SYT1",
  "gene_name": "Synaptotagmin-1",
  "term_label": "regulation of calcium ion-dependent exocytosis",
  "term_id": "GO:0017158",
  "gene": "UniProtKB:P21579"
}